{
  "gene_name": "Serine_threonine-protein phosphatase 2A 65 kDa regulatory subunit A alpha isoform",
  "term_label": "nucleus",
  "gene": "UniProtKB:P30153",
  "term_id": "GO:0005634",
  "gene_symbol": "PPP2R1A"
}